{
  "gene_symbol": "TDGF1",
  "gene": "UniProtKB:P13385",
  "term_id": "GO:0038100",
  "gene_name": "Teratocarcinoma-derived growth factor 1",
  "term_label": "nodal binding"
}